{
  "term_label": "protein-macromolecule adaptor activity",
  "gene_name": "FMR1-interacting protein NUFIP1",
  "term_id": "GO:0030674",
  "gene_symbol": "NUFIP1",
  "gene": "UniProtKB:Q9UHK0"
}